{
  "gene_name": "RING-box protein 2",
  "gene_symbol": "RNF7",
  "term_id": "GO:0097602",
  "term_label": "cullin family protein binding",
  "gene": "UniProtKB:Q9UBF6"
}